{
  "term_id": "GO:0098609",
  "term_label": "cell-cell adhesion",
  "gene_symbol": "ITGAX",
  "gene": "UniProtKB:P20702",
  "gene_name": "Integrin alpha-X"
}